negative regulation of kidney smooth muscle cell differentiation [GO:2000357] (biological process) Relationships: is a type of negative regulation of smooth muscle cell differentiation [GO:0051151]; is a type of regulation of kidney smooth muscle cell differentiation [GO:2000356]; negatively regulates GO:0072195 Definition: Any process that stops, prevents or reduces the frequency, rate or extent of kidney smooth muscle cell differentiation. Sources: GOC:obol